{
  "term_id": "UNKNOWN:0002",
  "gene": "UniProtKB:A0PJW6",
  "gene_name": "Transmembrane protein 223",
  "gene_symbol": "TMEM223",
  "term_label": "Unknown biological process"
}